3,5-dichloro-THPH methyl transferase activity [GO:0106268] (molecular function) Also known as: DIF-1 syntase Definition: Catalysis of the reaction: (3,5-dichloro-2,4,6-trihydroxyphenyl)hexan-1-one + S-adenosyl-L-methionine = 1-(3,5-dichloro-2,6-dihydroxy-4-methoxyphenyl)hexan-1-one + H+ + S-adenosyl-L-homocysteine. Relationships: is a type of S-adenosylmethionine-dependent methyltransferase activity [GO:0008757] References: PMID:20231486 Sources: RHEA:48396